{
  "gene": "UniProtKB:Q9Y6G1",
  "gene_symbol": "TMEM14A",
  "term_id": "UNKNOWN:0002",
  "gene_name": "Transmembrane protein 14A",
  "term_label": "Unknown biological process"
}